{
  "term_id": "GO:0005770",
  "gene_symbol": "SNX16",
  "gene_name": "Sorting nexin-16",
  "term_label": "late endosome",
  "gene": "UniProtKB:P57768"
}